{
  "gene": "UniProtKB:B1ATL7",
  "term_label": "Unknown biological process",
  "gene_name": "Proline-rich protein 32",
  "gene_symbol": "PRR32",
  "term_id": "UNKNOWN:0002"
}